negative regulation of mesenchymal to epithelial transition involved in metanephros morphogenesis [GO:0003340] (biological process) Definition: Any process that decreases the rate, frequency or extent of the transition where a mesenchymal cell establishes apical/basolateral polarity,forms intercellular adhesive junctions, synthesizes basement membrane components and becomes an epithelial cell that will contribute to the shaping of the metanephros. Sources: GOC:dph, GOC:yaf Relationships: is a type of regulation of mesenchymal to epithelial transition involved in metanephros morphogenesis [GO:0003339]; is a type of GO:2000697; negatively regulates mesenchymal to epithelial transition involved in metanephros morphogenesis [GO:0003337]